{
  "term_label": "Unknown molecular function",
  "term_id": "UNKNOWN:0001",
  "gene_name": "Cell growth regulator with RING finger domain protein 1",
  "gene_symbol": "CGRRF1",
  "gene": "UniProtKB:Q99675"
}